{
  "term_id": "GO:0005886",
  "gene_name": "Proteinase-activated receptor 2",
  "gene": "UniProtKB:P55085",
  "gene_symbol": "F2RL1",
  "term_label": "plasma membrane"
}